negative regulation of collateral sprouting in absence of injury [GO:0048698] (biological process) Definition: Any process that stops, prevents, or reduces the frequency, rate or extent of collateral sprouting in the absence of injury. Relationships: is a type of negative regulation of collateral sprouting [GO:0048671]; is a type of regulation of collateral sprouting in absence of injury [GO:0048696]; negatively regulates GO:0048669 Also known as: down regulation of collateral sprouting in the absence of injury, down-regulation of collateral sprouting in the absence of injury, downregulation of collateral sprouting in the absence of injury, inhibition of collateral sprouting in the absence of injury Sources: GOC:dgh, GOC:dph, GOC:jid, GOC:lm